{
  "gene_symbol": "ADAMTS19",
  "gene": "UniProtKB:Q8TE59",
  "gene_name": "A disintegrin and metalloproteinase with thrombospondin motifs 19",
  "term_id": "GO:0004222",
  "term_label": "metalloendopeptidase activity"
}